{
  "gene": "UniProtKB:O94819",
  "term_label": "Unknown biological process",
  "term_id": "UNKNOWN:0002",
  "gene_symbol": "KBTBD11",
  "gene_name": "Kelch repeat and BTB domain-containing protein 11"
}